negative regulation of bleb assembly [GO:1904171] (biological process) Definition: Any process that stops, prevents or reduces the frequency, rate or extent of bleb assembly. References: PMID:25651887 Sources: GOC:TermGenie, GOC:als, GO_REF:0000058 Relationships: is_a GO:0120033; is a type of regulation of bleb assembly [GO:1904170]; negatively regulates GO:0032060 Also known as: down regulation of bleb assembly, down regulation of cell blebbing, down-regulation of bleb assembly, down-regulation of cell blebbing, downregulation of bleb assembly, downregulation of cell blebbing, negative regulation of cell blebbing, inhibition of bleb assembly, inhibition of cell blebbing